{
  "gene_symbol": "RRAGD",
  "term_label": "nucleus",
  "gene_name": "Ras-related GTP-binding protein D",
  "gene": "UniProtKB:Q9NQL2",
  "term_id": "GO:0005634"
}